{
  "term_id": "GO:0051087",
  "gene_name": "TSSK6-activating co-chaperone protein",
  "term_label": "protein-folding chaperone binding",
  "gene_symbol": "TSACC",
  "gene": "UniProtKB:Q96A04"
}